4-aminobutyrate:2-oxoglutarate transaminase activity [GO:0034386] (molecular function) Also known as: 4-aminobutanoate:2-oxoglutarate aminotransferase activity, 4-aminobutyrate-2-ketoglutarate aminotransferase activity, 4-aminobutyrate-2-oxoglutarate aminotransferase activity, 4-aminobutyrate-2-oxoglutarate transaminase activity, 4-aminobutyric acid 2-ketoglutaric acid aminotransferase activity, GABA-2-oxoglutarate aminotransferase activity, GABA-2-oxoglutarate transaminase activity, GABA-alpha-ketoglutarate aminotransferase activity, GABA-alpha-ketoglutarate transaminase activity, GABA-alpha-ketoglutaric acid transaminase activity, GABA-alpha-oxoglutarate aminotransferase activity, GABA-oxoglutarate aminotransferase activity, GABA-oxoglutarate transaminase activity, gamma-aminobutyrate-alpha-ketoglutarate aminotransferase activity, gamma-aminobutyrate-alpha-ketoglutarate transaminase activity, gamma-aminobutyrate:alpha-oxoglutarate aminotransferase activity, gamma-aminobutyric acid-2-oxoglutarate transaminase activity, gamma-aminobutyric acid-alpha-ketoglutarate transaminase activity, gamma-aminobutyric acid-alpha-ketoglutaric acid aminotransferase activity Definition: Catalysis of the reaction: 2-oxoglutarate + 4-aminobutanoate = L-glutamate + succinate semialdehyde. Relationships: is a type of transaminase activity [GO:0008483] Sources: RHEA:23352